{
  "gene": "UniProtKB:P51532",
  "gene_name": "Transcription activator BRG1",
  "term_id": "GO:0000785",
  "term_label": "chromatin",
  "gene_symbol": "SMARCA4"
}